{
  "term_label": "precatalytic spliceosome",
  "gene": "UniProtKB:P55769",
  "gene_symbol": "SNU13",
  "term_id": "GO:0071011",
  "gene_name": "NHP2-like protein 1"
}